{
  "gene": "UniProtKB:Q9BZD7",
  "term_id": "GO:0006508",
  "gene_name": "Transmembrane gamma-carboxyglutamic acid protein 3",
  "gene_symbol": "PRRG3",
  "term_label": "proteolysis"
}